{
  "gene_symbol": "CCER1",
  "gene": "UniProtKB:Q8TC90",
  "term_id": "UNKNOWN:0001",
  "gene_name": "Coiled-coil domain-containing glutamate-rich protein 1",
  "term_label": "Unknown molecular function"
}